pheromone receptor activity [GO:0016503] (molecular function) Sources: GOC:hjd, ISBN:0198506732 Relationships: is_a G protein-coupled receptor activity [GO:0004930]; has part pheromone binding [GO:0005550] Definition: Combining with a pheromone to initiate a change in cell activity. A pheromone is a substance used in olfactory communication between organisms of the same species eliciting a change in sexual or social behavior. Subtypes: mating-type factor pheromone receptor activity [GO:0004932], GO:0036318